positive regulation of interleukin-17-mediated signaling pathway [GO:1903883] (biological process) Also known as: positive regulation of IL-17-mediated signaling pathway, positive regulation of IL-17-mediated signalling pathway, positive regulation of interleukin-17-mediated signalling pathway, up regulation of IL-17-mediated signaling pathway, up regulation of IL-17-mediated signalling pathway, up regulation of interleukin-17-mediated signaling pathway, up regulation of interleukin-17-mediated signalling pathway, up-regulation of IL-17-mediated signaling pathway, up-regulation of IL-17-mediated signalling pathway, up-regulation of interleukin-17-mediated signaling pathway, up-regulation of interleukin-17-mediated signalling pathway, upregulation of IL-17-mediated signaling pathway, upregulation of IL-17-mediated signalling pathway, upregulation of interleukin-17-mediated signaling pathway, upregulation of interleukin-17-mediated signalling pathway, activation of IL-17-mediated signaling pathway, activation of IL-17-mediated signalling pathway, activation of interleukin-17-mediated signaling pathway, activation of interleukin-17-mediated signalling pathway Relationships: is a type of positive regulation of cytokine-mediated signaling pathway [GO:0001961]; is a type of regulation of interleukin-17-mediated signaling pathway [GO:1903881]; positively regulates interleukin-17-mediated signaling pathway [GO:0097400] Definition: Any process that activates or increases the frequency, rate or extent of interleukin-17-mediated signaling pathway. References: PMID:20054338 Sources: GOC:TermGenie, GOC:krc, GO_REF:0000058